{
  "gene": "UniProtKB:Q8IVL1",
  "term_id": "GO:0007399",
  "gene_name": "Neuron navigator 2",
  "gene_symbol": "NAV2",
  "term_label": "nervous system development"
}